{
  "gene": "UniProtKB:P67809",
  "gene_name": "Y-box-binding protein 1",
  "gene_symbol": "YBX1",
  "term_label": "nucleic acid binding",
  "term_id": "GO:0003676"
}